{
  "gene": "UniProtKB:P35670",
  "gene_symbol": "ATP7B",
  "term_label": "copper ion import",
  "gene_name": "Copper-transporting ATPase 2",
  "term_id": "GO:0015677"
}